{
  "term_id": "GO:0005634",
  "gene": "UniProtKB:Q96NX9",
  "gene_name": "Dachshund homolog 2",
  "gene_symbol": "DACH2",
  "term_label": "nucleus"
}